{
  "gene_symbol": "GLS2",
  "term_label": "L-glutamine catabolic process",
  "gene_name": "Glutaminase liver isoform, mitochondrial",
  "term_id": "GO:0006543",
  "gene": "UniProtKB:Q9UI32"
}